{
  "term_label": "extracellular space",
  "gene_name": "Complement component C9",
  "term_id": "GO:0005615",
  "gene_symbol": "C9",
  "gene": "UniProtKB:P02748"
}